protein localization to extracellular region [GO:0071692] (biological process) Definition: Any process in which a protein is transported from one specific location in the extracellular region to another, or maintained in a specific extracellular location. Sources: GOC:mah Relationships: is a type of macromolecule localization [GO:0033036] Subtypes: protein secretion [GO:0009306], GO:0071693 Also known as: protein localisation in extracellular region, protein localization in extracellular region